dityrosine layer of spore wall [GO:0005630] (cellular component) Relationships: is a type of GO:0110165; is part of ascospore wall [GO:0005619] Sources: ISBN:0879693568 Definition: The outermost layer of the spore wall, as described in Saccharomyces.